mesonephric glomerular basement membrane development [GO:0061233] (biological process) Sources: GOC:mtg_kidney_jan10 Relationships: is a type of glomerular basement membrane development [GO:0032836]; is part of mesonephric glomerulus development [GO:0061224] Definition: The process whose specific outcome is the progression of the mesonephric glomerular basement membrane over time, from its formation to the mature structure. The mesonephric glomerular basement membrane is the basal laminal portion of the mesonephric glomerulus which performs the actual filtration.